{
  "gene_name": "Serine_threonine-protein kinase DCLK2",
  "gene": "UniProtKB:Q8N568",
  "term_label": "microtubule cytoskeleton organization",
  "gene_symbol": "DCLK2",
  "term_id": "GO:0000226"
}